{
  "term_label": "nucleus",
  "term_id": "GO:0005634",
  "gene_name": "Jerky protein homolog",
  "gene_symbol": "JRK",
  "gene": "UniProtKB:O75564"
}